{
  "term_id": "GO:0005737",
  "term_label": "cytoplasm",
  "gene": "UniProtKB:P17050",
  "gene_symbol": "NAGA",
  "gene_name": "Alpha-N-acetylgalactosaminidase"
}